{
  "gene_name": "Probable helicase senataxin",
  "term_id": "GO:0006369",
  "term_label": "termination of RNA polymerase II transcription",
  "gene": "UniProtKB:Q7Z333",
  "gene_symbol": "SETX"
}